mitotic nuclear pore complex disassembly [GO:0140516] (biological process) Relationships: is a type of nuclear pore organization [GO:0006999]; is a type of mitotic nuclear membrane disassembly [GO:0007077]; is a type of GO:0032984 Definition: The mitotic cell cycle process in which the controlled breakdown of the nuclear pores occurs during open or closed mitosis. References: PMID:32848252 Also known as: nuclear pore complex disassembly during mitosis